{
  "gene_name": "Core histone macro-H2A.2",
  "gene": "UniProtKB:Q9P0M6",
  "term_id": "GO:0030527",
  "gene_symbol": "MACROH2A2",
  "term_label": "structural constituent of chromatin"
}